glutathione hydrolase complex [GO:0061672] (cellular component) Relationships: is a type of peptidase complex [GO:1905368] Also known as: gamma-glutamyltranspeptidase complex, glutathionase complex, glutamine amidotransferase II complex Sources: GOC:dph Definition: Enzyme complex that in S. cerevisiae has components Dug2/Dug3 and is able to catalyze the cleavage of glutathione into glutamate and Cys-Gly.